{
  "term_id": "UNKNOWN:0003",
  "gene_symbol": "FN3K",
  "gene_name": "Fructosamine-3-kinase",
  "term_label": "Unknown cellular component",
  "gene": "UniProtKB:Q9H479"
}